2-hydroxy-3-keto-5-methylthiopentenyl-1-phosphate phosphatase activity [GO:0043716] (MF) Sources: RHEA:14481 Also known as: 2-hydroxy-3-keto-5-methylthio-phosphopentene phosphatase activity, HK-MTPenyl-1-P phosphatase activity Relationships: is a type of phosphatase activity [GO:0016791] Definition: Catalysis of the reaction: 2-hydroxy-5-methylsulfanyl-3-oxopent-1-enyl phosphate + H2O = 1,2-dihydroxy-5-(methylsulfanyl)pent-1-en-3-one + phosphate.